positive regulation of toll-like receptor 1 signaling pathway [GO:0034133] (BP) Definition: Any process that activates or increases the frequency, rate, or extent of toll-like receptor 1 signaling pathway. References: PMID:16551253, PMID:17328678 Sources: GOC:add Also known as: positive regulation of TLR1 signaling pathway, positive regulation of toll-like receptor 1 signalling pathway Relationships: is_a regulation of toll-like receptor 1 signaling pathway [GO:0034131]; is a type of GO:0062208; positively regulates GO:0034130